pituitary adenylate cyclase activating polypeptide activity [GO:0016521] (molecular function) Definition: The action characteristic of pituitary adenylate cyclase activating polypeptide, a peptide produced in the hypothalamus that binds to receptors to exert pleiotropic effects including control of neurotransmitter release, vasodilation, bronchodilation, activation of intestinal motility, increase in insulin and histamine secretion, immune modulation, and stimulation of cell proliferation and differentiation. Also known as: pituitary adenylyl cyclase activating polypeptide activity Relationships: is a type of hormone activity [GO:0005179] References: PMID:19805477 Sources: GOC:mah